asymmetric neuroblast division resulting in ganglion mother cell formation [GO:0055060] (biological process) Sources: GOC:dph Relationships: is a type of neuroblast fate commitment [GO:0014017]; is a type of GO:0055059 Definition: Any process resulting in the physical partitioning and separation of a neuroblast into a neuroblast and a ganglion mother cell.